regulation of tolerance induction to nonself antigen [GO:0002655] (biological process) Definition: Any process that modulates the frequency, rate, or extent of tolerance induction to nonself antigen. Subtypes: negative regulation of tolerance induction to nonself antigen [GO:0002656], positive regulation of tolerance induction to nonself antigen [GO:0002657] Sources: GOC:add Relationships: is_a GO:0002652; regulates tolerance induction to nonself antigen [GO:0002462]